cell surface furrow [GO:0097610] (cellular component) Subtypes: dinoflagellate cingulum [GO:0097611], dinoflagellate sulcus [GO:0097612], dinoflagellate apical groove [GO:0097685] Definition: A furrow that may be found on the cell surface. Examples include the cingulum and sulcus found in some dinoflagellates. Sources: GOC:pr Also known as: furrow, groove, cell surface groove Relationships: is a type of cellular anatomical structure [GO:0110165]; is part of cell surface [GO:0009986]